positive regulation of T-helper 2 cell cytokine production [GO:2000553] (biological process) Relationships: is_a positive regulation of T cell cytokine production [GO:0002726]; is a type of positive regulation of type 2 immune response [GO:0002830]; is a type of regulation of T-helper 2 cell cytokine production [GO:2000551]; positively regulates T-helper 2 cell cytokine production [GO:0035745] Definition: Any process that activates or increases the frequency, rate or extent of T-helper 2 cell cytokine production. Also known as: positive regulation of Th2 cell cytokine production Sources: GOC:obol